{
  "term_id": "UNKNOWN:0001",
  "gene": "UniProtKB:Q9Y4I5",
  "gene_symbol": "TESMIN",
  "gene_name": "Tesmin",
  "term_label": "Unknown molecular function"
}